{
  "term_id": "GO:0007218",
  "gene_name": "Neuropeptides B_W receptor type 1",
  "gene_symbol": "NPBWR1",
  "gene": "UniProtKB:P48145",
  "term_label": "neuropeptide signaling pathway"
}